D-arabinose catabolic process to D-xylulose 5-phosphate [GO:0019573] (biological process) Also known as: D-arabinose breakdown to xylulose 5-phosphate, D-arabinose degradation to xylulose 5-phosphate Relationships: is a type of D-arabinose catabolic process [GO:0019571]; is_a D-xylulose 5-phosphate metabolic process [GO:0051167] Sources: GOC:go_curators Definition: The chemical reactions and pathways resulting in the breakdown of D-arabinose to form D-xylulose 5-phosphate. D-arabinose is converted into D-ribulose, which is phosphorylated to D-ribulose-5-phosphate, which is isomerized to give D-xylulose-5-phosphate.